{
  "gene_name": "Oxygen-dependent coproporphyrinogen-III oxidase, mitochondrial",
  "term_label": "coproporphyrinogen oxidase activity",
  "term_id": "GO:0004109",
  "gene": "UniProtKB:P36551",
  "gene_symbol": "CPOX"
}